{
  "gene_symbol": "U2SURP",
  "gene_name": "U2 snRNP-associated SURP motif-containing protein",
  "gene": "UniProtKB:O15042",
  "term_id": "GO:0003723",
  "term_label": "RNA binding"
}